{
  "gene_symbol": "MYO7B",
  "term_id": "GO:0007423",
  "term_label": "sensory organ development",
  "gene": "UniProtKB:Q6PIF6",
  "gene_name": "Unconventional myosin-VIIb"
}